{
  "gene": "UniProtKB:Q8WTR4",
  "gene_symbol": "GDPD5",
  "term_id": "GO:0045666",
  "gene_name": "Glycerophosphodiester phosphodiesterase domain-containing protein 5",
  "term_label": "positive regulation of neuron differentiation"
}